{
  "term_id": "GO:0045294",
  "gene_name": "Junction plakoglobin",
  "term_label": "alpha-catenin binding",
  "gene_symbol": "JUP",
  "gene": "UniProtKB:P14923"
}